{
  "gene": "UniProtKB:Q8N2W9",
  "term_id": "GO:0061665",
  "term_label": "SUMO ligase activity",
  "gene_name": "E3 SUMO-protein ligase PIAS4",
  "gene_symbol": "PIAS4"
}